{
  "term_label": "proton transmembrane transport",
  "gene_symbol": "SLC36A3",
  "gene_name": "Proton-coupled amino acid transporter 3",
  "term_id": "GO:1902600",
  "gene": "UniProtKB:Q495N2"
}